{
  "gene_symbol": "EIF3I",
  "term_id": "GO:0003723",
  "term_label": "RNA binding",
  "gene_name": "Eukaryotic translation initiation factor 3 subunit I",
  "gene": "UniProtKB:Q13347"
}